regulation of acute inflammatory response to antigenic stimulus [GO:0002864] (biological process) Definition: Any process that modulates the frequency, rate, or extent of an acute inflammatory response to an antigenic stimulus. Sources: GOC:add Relationships: is a type of regulation of acute inflammatory response [GO:0002673]; is_a GO:0002861; regulates acute inflammatory response to antigenic stimulus [GO:0002438] Subtypes: negative regulation of acute inflammatory response to antigenic stimulus [GO:0002865], positive regulation of acute inflammatory response to antigenic stimulus [GO:0002866], GO:0002883